{
  "gene_name": "UDP-glucuronosyltransferase 2A3",
  "term_label": "glucuronosyltransferase activity",
  "gene": "UniProtKB:Q6UWM9",
  "gene_symbol": "UGT2A3",
  "term_id": "GO:0015020"
}